{
  "gene_name": "RING finger and transmembrane domain-containing protein 2",
  "term_label": "Unknown biological process",
  "term_id": "UNKNOWN:0002",
  "gene_symbol": "RNFT2",
  "gene": "UniProtKB:Q96EX2"
}